{
  "term_label": "plasma membrane",
  "gene_symbol": "SYT13",
  "term_id": "GO:0005886",
  "gene": "UniProtKB:Q7L8C5",
  "gene_name": "Synaptotagmin-13"
}